{
  "gene_symbol": "GHSR",
  "term_label": "growth hormone secretagogue receptor activity",
  "term_id": "GO:0001616",
  "gene_name": "Growth hormone secretagogue receptor type 1",
  "gene": "UniProtKB:Q92847"
}